{
  "term_label": "G protein-coupled receptor signaling pathway",
  "gene_name": "Growth hormone secretagogue receptor type 1",
  "term_id": "GO:0007186",
  "gene_symbol": "GHSR",
  "gene": "UniProtKB:Q92847"
}